sugar-phosphatase activity [GO:0050308] (molecular function) Subtypes: 2-deoxyglucose-6-phosphatase activity [GO:0003850], GO:0004331, GO:0004805, glucose-1-phosphatase activity [GO:0008877], fructose 1,6-bisphosphate 1-phosphatase activity [GO:0042132], GO:0047386, sucrose-phosphate phosphatase activity [GO:0050307], sugar-terminal-phosphatase activity [GO:0050309], galactose-1-phosphate phosphatase activity [GO:0070456] Also known as: sugar-phosphate phosphatase activity, sugar-phosphate phosphohydrolase activity Sources: EC:3.1.3.23, MetaCyc:SUGAR-PHOSPHATASE-RXN Relationships: is a type of carbohydrate phosphatase activity [GO:0019203] Definition: Catalysis of the reaction: sugar phosphate + H2O = sugar + phosphate.